{
  "gene": "UniProtKB:Q9BYX7",
  "gene_symbol": "POTEKP",
  "gene_name": "Putative beta-actin-like protein 3",
  "term_label": "cytoplasm",
  "term_id": "GO:0005737"
}